{
  "gene_symbol": "CCM2L",
  "gene_name": "Cerebral cavernous malformations 2 protein-like",
  "term_id": "UNKNOWN:0001",
  "term_label": "Unknown molecular function",
  "gene": "UniProtKB:Q9NUG4"
}